{
  "term_id": "GO:0005789",
  "gene": "UniProtKB:Q8NCC5",
  "gene_name": "Sugar phosphate exchanger 3",
  "gene_symbol": "SLC37A3",
  "term_label": "endoplasmic reticulum membrane"
}